histone H3K9ac reader activity [GO:0140072] (molecular function) Definition: A histone reader that recognizes a histone H3 acetylated at lysine 9. Note: Comment: Note that the residue position corresponds to the canonical human H3 histone (UniProtKB:P84243); this residue is conserved across all eukaryotes. Residue 1 is the first residue following removal of the initiating Methionine (Met). Note that each histone is encoded by multiple genes, and sequences may vary across different genes within an organism. References: PMID:26067602 Also known as: H3K9ac modified histone binding Relationships: is a type of GO:0140006